negative regulation of pentose-phosphate shunt [GO:1905856] (biological process) Definition: Any process that stops, prevents or reduces the frequency, rate or extent of pentose-phosphate shunt. References: PMID:19015259 Sources: GOC:TermGenie, GO_REF:0000058 Relationships: is a type of regulation of pentose-phosphate shunt [GO:0043456]; is a type of GO:1900543; negatively regulates GO:0006098